zinc potentiation of synaptic transmission, glycinergic [GO:0060095] (biological process) Definition: Any process that activates or increases the frequency, rate or extent of glycinergic synaptic transmission in the presence of zinc. Glycinergic synaptic transmission is the process of communication from a neuron to another neuron across a synapse using the neurotransmitter glycine. Also known as: zinc potentiation of glycinergic synaptic transmission Relationships: is a type of positive regulation of synaptic transmission, glycinergic [GO:0060094] Sources: GOC:dms, GOC:dph